collagen type XIII trimer [GO:0005600] (cellular component) Relationships: is a type of GO:0030936 References: PMID:21421911 Definition: A collagen homotrimer of alpha1(XIII) chains; type XIII collagen triple helices span the plasma membrane.